{
  "gene_symbol": "MRFAP1",
  "gene_name": "MORF4 family-associated protein 1",
  "term_label": "Unknown cellular component",
  "term_id": "UNKNOWN:0003",
  "gene": "UniProtKB:Q9Y605"
}